{
  "gene_name": "Small cysteine and glycine repeat-containing protein 8",
  "term_label": "Unknown molecular function",
  "gene": "UniProtKB:A0A286YFG1",
  "gene_symbol": "SCYGR8",
  "term_id": "UNKNOWN:0001"
}